{
  "gene_name": "B2 bradykinin receptor",
  "gene": "UniProtKB:P30411",
  "gene_symbol": "BDKRB2",
  "term_id": "GO:0005886",
  "term_label": "plasma membrane"
}